CRD-mediated mRNA stabilization [GO:0070934] (biological process) Definition: An mRNA stabilization process in which one or more RNA-binding proteins associate with a sequence in the open reading frame called the coding region instability determinant (CRD). Also known as: coding region determinant-mediated mRNA stabilization References: PMID:19029303 Sources: GOC:mah Relationships: is a type of GO:0048255